alpha-L-rhamnosidase activity [GO:0030596] (molecular function) Also known as: alpha-L-rhamnosidase N, alpha-L-rhamnosidase T, alpha-L-rhamnoside rhamnohydrolase activity Definition: Catalysis of the hydrolysis of terminal non-reducing alpha-L-rhamnose residues in alpha-L-rhamnosides. Relationships: is a type of hydrolase activity, hydrolyzing O-glycosyl compounds [GO:0004553] Sources: EC:3.2.1.40